{
  "gene_symbol": "AVPR2",
  "term_label": "cellular response to hormone stimulus",
  "term_id": "GO:0032870",
  "gene_name": "Vasopressin V2 receptor",
  "gene": "UniProtKB:P30518"
}